{
  "gene": "UniProtKB:Q5T0D9",
  "gene_name": "Tumor protein p63-regulated gene 1-like protein",
  "gene_symbol": "TPRG1L",
  "term_id": "UNKNOWN:0001",
  "term_label": "Unknown molecular function"
}